{
  "gene": "UniProtKB:Q9C0K0",
  "term_id": "GO:0005634",
  "term_label": "nucleus",
  "gene_name": "B-cell lymphoma_leukemia 11B",
  "gene_symbol": "BCL11B"
}